{
  "gene": "UniProtKB:Q9Y4B5",
  "term_id": "GO:0016328",
  "gene_symbol": "MTCL1",
  "gene_name": "Microtubule cross-linking factor 1",
  "term_label": "lateral plasma membrane"
}